2-C-methyl-D-erythritol 2,4-cyclodiphosphate synthase activity [GO:0008685] (molecular function) Definition: Catalysis of the reaction: 4-CDP-2-C-methyl-D-erythritol 2-phosphate = 2-C-methyl-D-erythritol 2,4-cyclic diphosphate + CMP. Sources: EC:4.6.1.12, RHEA:23864 Also known as: MECP synthase activity, 2-phospho-4-(cytidine 5'-diphospho)-2-C-methyl-D-erythritol CMP-lyase (cyclizing), 2-phospho-4-(cytidine 5'-diphospho)-2-C-methyl-D-erythritol CMP-lyase (cyclizing; 2-C-methyl-D-erythritol 2,4-cyclodiphosphate-forming), MECDP-synthase activity Relationships: is a type of phosphorus-oxygen lyase activity [GO:0016849]